serine C-palmitoyltransferase activity [GO:0004758] (molecular function) Definition: Catalysis of the reaction: L-serine + H+ + palmitoyl-CoA = 3-dehydrosphinganine + CO2 + CoA. Regulation: positively regulated by positive regulation of serine C-palmitoyltransferase activity [GO:1904222] Relationships: is a type of C-palmitoyltransferase activity [GO:0016454] Sources: EC:2.3.1.50, RHEA:14761 Also known as: serine palmitoyltransferase, 3-oxosphinganine synthetase activity, SPT